{
  "gene_symbol": "SLC7A1",
  "term_label": "L-ornithine transmembrane transport",
  "term_id": "GO:1903352",
  "gene_name": "High affinity cationic amino acid transporter 1",
  "gene": "UniProtKB:P30825"
}